{
  "gene": "UniProtKB:P55774",
  "term_id": "GO:0060326",
  "gene_name": "C-C motif chemokine 18",
  "gene_symbol": "CCL18",
  "term_label": "cell chemotaxis"
}